{
  "term_id": "GO:0036064",
  "gene_name": "Intraflagellar transport protein 172 homolog",
  "gene_symbol": "IFT172",
  "gene": "UniProtKB:Q9UG01",
  "term_label": "ciliary basal body"
}